import across plasma membrane [GO:0098739] (biological process) Sources: GOC:dos Definition: The directed movement of some substance from outside of a cell, across the plasma membrane and into the cytosol. Relationships: is a type of transmembrane transport [GO:0055085]; is a type of import into cell [GO:0098657] Subtypes: long-chain fatty acid import across plasma membrane [GO:0015911], auxin import into cell [GO:0060919], amino acid import across plasma membrane [GO:0089718], adenine import across plasma membrane [GO:0098702], carbohydrate import across plasma membrane [GO:0098704], GO:0098710, malate import across plasma membrane [GO:0098714], malonic acid import across plasma membrane [GO:0098715], pantothenate import across plasma membrane [GO:0098717], succinate import across plasma membrane [GO:0098720], GO:0098721, inorganic ion import across plasma membrane [GO:0099587], thiamine import across plasma membrane [GO:0140125], GO:0140201, polyamine import across plasma membrane [GO:0140202], pyridoxal import across plasma membrane [GO:0140204], oligopeptide import across plasma membrane [GO:0140205], GO:0140270, cyclic-GMP-AMP transmembrane import across plasma membrane [GO:0140361], GO:0160284, queuosine import across plasma membrane [GO:0160287], nucleoside import across plasma membrane [GO:0180015], pyridoxine import across plasma membrane [GO:1903075], folate import across plasma membrane [GO:1904447], myo-inositol import across plasma membrane [GO:1904679], GO:1905130, biotin import across plasma membrane [GO:1905135], dethiobiotin import across plasma membrane [GO:1905136] Also known as: uptake